{
  "gene": "UniProtKB:P41145",
  "term_label": "plasma membrane",
  "gene_name": "Kappa-type opioid receptor",
  "term_id": "GO:0005886",
  "gene_symbol": "OPRK1"
}